{
  "term_id": "GO:0031386",
  "term_label": "protein tag activity",
  "gene": "UniProtKB:P55854",
  "gene_name": "Small ubiquitin-related modifier 3",
  "gene_symbol": "SUMO3"
}